{
  "gene_name": "MORC family CW-type zinc finger protein 1",
  "term_label": "nucleus",
  "gene": "UniProtKB:Q86VD1",
  "gene_symbol": "MORC1",
  "term_id": "GO:0005634"
}